endopeptidase Clp complex [GO:0009368] (cellular component) Subtypes: chloroplastic endopeptidase Clp complex [GO:0009840], mitochondrial endopeptidase Clp complex [GO:0009841] References: PMID:11352464 Sources: GOC:mah Relationships: is a type of catalytic complex [GO:1902494] Definition: A protein complex comprised of members of the ClpX, ClpC, ClpD, ClpP or ClpR protein families. ClpPs are the proteolytic subunit of active complexes, and ClpA and ClpX form the regulatory subunits. Enzymatically active and inactive complexes can form.